{
  "term_label": "Unknown biological process",
  "gene_symbol": "GPR158",
  "gene": "UniProtKB:Q5T848",
  "term_id": "UNKNOWN:0002",
  "gene_name": "Probable G-protein coupled receptor 158"
}